establishment or maintenance of cytoskeleton polarity involved in gastrulation [GO:0003380] (biological process) Subtypes: establishment or maintenance of cytoskeleton polarity involved in mesendodermal cell migration [GO:0003372] Relationships: is a type of establishment or maintenance of cytoskeleton polarity involved in ameboidal cell migration [GO:0003371]; is part of establishment of cell polarity involved in gastrulation cell migration [GO:0003379] Definition: Any cellular process that results in the specification, formation or maintenance of polarized cytoskeletal structures that contribute to the cell polarity of a migrating ameboid cell taking part in gastrulation. Sources: GOC:ascb_2009, GOC:dph, GOC:tb